{
  "gene_name": "V-set and transmembrane domain-containing protein 2B",
  "term_label": "membrane",
  "gene": "UniProtKB:A6NLU5",
  "gene_symbol": "VSTM2B",
  "term_id": "GO:0016020"
}